plant epidermal cell fate specification [GO:0090628] (biological process) Relationships: is a type of cell fate specification [GO:0001708]; is part of GO:0090627 Sources: GOC:tb Subtypes: atrichoblast fate specification [GO:0010056], trichoblast fate specification [GO:0010057] Definition: The process in which a cell becomes capable of differentiating autonomously into a plant epidermal cell in an environment that is neutral with respect to the developmental pathway. Upon specification, the cell fate can be reversed.